{
  "gene_symbol": "SLC35E3",
  "gene_name": "Solute carrier family 35 member E3",
  "gene": "UniProtKB:Q7Z769",
  "term_id": "GO:0005338",
  "term_label": "nucleotide-sugar transmembrane transporter activity"
}